{
  "gene": "UniProtKB:P01275",
  "term_id": "GO:0035774",
  "term_label": "positive regulation of insulin secretion involved in cellular response to glucose stimulus",
  "gene_name": "Pro-glucagon",
  "gene_symbol": "GCG"
}